acetyltransferase activity [GO:0016407] (molecular function) Definition: Catalysis of the transfer of an acetyl group to an acceptor molecule. Sources: GOC:ai Also known as: acetylase activity Relationships: is a type of acyltransferase activity, transferring groups other than amino-acyl groups [GO:0016747] Subtypes: N-acetyltransferase activity [GO:0008080], phosphate acetyltransferase activity [GO:0008959], O-acetyltransferase activity [GO:0016413], S-acetyltransferase activity [GO:0016418], GO:0016453, diaminobutyrate acetyltransferase activity [GO:0033816], GO:0043894, platelet-activating factor acetyltransferase activity [GO:0047179], tRNA uridine(34) acetyltransferase activity [GO:0106261] Regulation: positively regulated by acetyltransferase activator activity [GO:0010698]